metanephric glomerular epithelium development [GO:0072244] (biological process) Sources: GOC:mtg_kidney_jan10 Definition: The process whose specific outcome is the progression of the metanephric glomerular epithelium over time, from its formation to the mature structure. The metanephric glomerular epithelium is an epithelial tissue that covers the outer surfaces of the glomerulus in the metanephros. The metanephric glomerular epithelium consists of both parietal and visceral epithelium. Metanephric glomerular parietal epithelial cells are specialized epithelial cells that form tight junctions as a barrier to protein transport. A metanephric glomerular visceral epithelial cell is a specialized epithelial cell that contains 'feet' that interdigitate with the 'feet' of other glomerular epithelial cells in the metanephros. Subtypes: metanephric glomerular endothelium development [GO:0072264] Relationships: is_a glomerular epithelium development [GO:0072010]; is a type of GO:0072243; is part of metanephric glomerulus development [GO:0072224]